{
  "term_label": "ubiquitin-like ligase-substrate adaptor activity",
  "gene_symbol": "KLHL20",
  "gene_name": "Kelch-like protein 20",
  "term_id": "GO:1990756",
  "gene": "UniProtKB:Q9Y2M5"
}